{
  "gene_name": "Mediator of RNA polymerase II transcription subunit 25",
  "term_label": "positive regulation of transcription by RNA polymerase II",
  "term_id": "GO:0045944",
  "gene": "UniProtKB:Q71SY5",
  "gene_symbol": "MED25"
}